type 1 metabotropic glutamate receptor binding [GO:0031798] (molecular function) Relationships: is a type of G protein-coupled glutamate receptor binding [GO:0035256] Sources: GOC:mah, GOC:nln Also known as: type 1 metabotropic glutamate receptor ligand Definition: Binding to a type 1 metabotropic glutamate receptor.